{
  "gene": "UniProtKB:P20333",
  "gene_symbol": "TNFRSF1B",
  "term_id": "GO:0051044",
  "term_label": "positive regulation of membrane protein ectodomain proteolysis",
  "gene_name": "Tumor necrosis factor receptor superfamily member 1B"
}